protein exit from endoplasmic reticulum [GO:0032527] (BP) Subtypes: retrograde protein transport, ER to cytosol [GO:0030970] Sources: GOC:rb Definition: The directed movement of proteins from the endoplasmic reticulum. Also known as: protein exit from ER, protein export from ER, protein export from endoplasmic reticulum Relationships: is a type of GO:0006886; occurs in GO:0005737 Regulation: regulated by regulation of protein exit from endoplasmic reticulum [GO:0070861]; negatively regulated by negative regulation of protein exit from endoplasmic reticulum [GO:0070862]; positively regulated by positive regulation of protein exit from endoplasmic reticulum [GO:0070863]